somatostatin secretion [GO:0070253] (biological process) Definition: The regulated release of somatostatin from secretory granules in the D cells of the pancreas. Sources: GOC:mah Relationships: is a type of peptide hormone secretion [GO:0030072] Regulation: regulated by GO:0090273; positively regulated by positive regulation of somatostatin secretion [GO:0090274]; negatively regulated by negative regulation of somatostatin secretion [GO:0090275]